{
  "term_id": "GO:0005832",
  "gene_name": "T-complex protein 1 subunit theta",
  "gene": "UniProtKB:P50990",
  "term_label": "chaperonin-containing T-complex",
  "gene_symbol": "CCT8"
}